{
  "gene_name": "Mitochondrial protein C2orf69",
  "gene_symbol": "C2orf69",
  "term_label": "Unknown biological process",
  "gene": "UniProtKB:Q8N8R5",
  "term_id": "UNKNOWN:0002"
}